{
  "term_label": "SNAP receptor activity",
  "gene_symbol": "STX11",
  "term_id": "GO:0005484",
  "gene": "UniProtKB:O75558",
  "gene_name": "Syntaxin-11"
}